regulation of bile acid biosynthetic process [GO:0070857] (biological process) Relationships: is a type of regulation of ketone metabolic process [GO:0010565]; is a type of regulation of steroid biosynthetic process [GO:0050810]; is_a regulation of small molecule metabolic process [GO:0062012]; regulates bile acid biosynthetic process [GO:0006699] Definition: Any process that modulates the frequency, rate or extent of the chemical reactions and pathways resulting in the formation of bile acids. Also known as: regulation of bile acid anabolism, regulation of bile acid biosynthesis, regulation of bile acid formation, regulation of bile acid synthesis Subtypes: negative regulation of bile acid biosynthetic process [GO:0070858], GO:0070859 Sources: GOC:BHF, GOC:mah